{
  "term_id": "GO:0016485",
  "gene_name": "Tolloid-like protein 1",
  "gene_symbol": "TLL1",
  "gene": "UniProtKB:O43897",
  "term_label": "protein processing"
}